protein autosumoylation [GO:1990466] (biological process) Also known as: protein auto-sumoylation, protein self-sumoylation Definition: The sumoylation by a protein of one or more of its own amino acid residues, or residues on an identical protein. References: PMID:21518767, PMID:23443663 Relationships: is a type of protein sumoylation [GO:0016925]